{
  "gene": "UniProtKB:P49447",
  "term_label": "lysosomal membrane",
  "term_id": "GO:0005765",
  "gene_symbol": "CYB561",
  "gene_name": "Transmembrane ascorbate-dependent reductase CYB561"
}